hyaluronan metabolic process [GO:0030212] (biological process) Subtypes: hyaluronan biosynthetic process [GO:0030213], hyaluronan catabolic process [GO:0030214] Also known as: hyaluronan metabolism Relationships: is a type of glycosaminoglycan metabolic process [GO:0030203] Definition: The chemical reactions and pathways involving hyaluronan, the naturally occurring anionic form of hyaluronic acid. Hyaluronan is a type of non-sulfated glycosaminoglycan composed of the repeating disaccharide unit beta(1,4)-D-glucuronic acid-beta(1,3)-N-acetyl-D-glucosamine. References: PMID:33171800, PMID:35536932